endosome membrane [GO:0010008] (cellular component) Definition: The lipid bilayer surrounding an endosome. Sources: GOC:mah Also known as: endosomal membrane Relationships: is_a cytoplasmic vesicle membrane [GO:0030659]; is a type of bounding membrane of organelle [GO:0098588]; is part of GO:0005768 Subtypes: early endosome membrane [GO:0031901], late endosome membrane [GO:0031902], endolysosome membrane [GO:0036020], recycling endosome membrane [GO:0055038], postsynaptic endosome membrane [GO:0098895], presynaptic endosome membrane [GO:0098954], macropinosome membrane [GO:0160056]